signal sequence binding [GO:0005048] (MF) Definition: Binding to a signal sequence, a specific peptide sequence found on protein precursors or mature proteins that dictates where the mature protein is localized. Sources: GOC:ai Also known as: leader sequence binding, protein signal sequence binding, signal sequence receptor Relationships: is a type of peptide binding [GO:0042277] Subtypes: peroxisome targeting sequence binding [GO:0000268], nuclear localization sequence binding [GO:0008139], vacuolar sorting signal binding [GO:0010209], GO:0030941, GO:0030942, GO:0030943, ER retention sequence binding [GO:0046923], ciliary targeting signal binding [GO:1990473]